GDF15-GFRAL signaling pathway [GO:0160144] (biological process) Regulation: negatively regulated by negative regulation of GDF15-GFRAL signaling pathway [GO:0160145] References: PMID:30639358, PMID:31535977, PMID:33593916, PMID:37437602 Relationships: is a type of cellular response to stress [GO:0033554]; is a type of GO:0035860 Definition: The series of molecular signals initiated by GDF15 binding to GFRAL coreceptor, triggering RET autophosphorylation and activation, in response to stress.